{
  "gene_symbol": "RNF103",
  "gene": "UniProtKB:O00237",
  "term_id": "GO:0005783",
  "term_label": "endoplasmic reticulum",
  "gene_name": "E3 ubiquitin-protein ligase RNF103"
}